glycolytic process from galactose [GO:0061623] (biological process) Relationships: is a type of galactose catabolic process [GO:0019388]; is a type of glycolytic process through glucose-1-phosphate [GO:0061622]; has part GO:0033499 Sources: GOC:dph, ISBN:0201090910 Definition: The chemical reactions and pathways resulting in the breakdown of galactose into pyruvate, with the concomitant production of a small amount of ATP.